{
  "term_id": "UNKNOWN:0003",
  "gene_name": "Uncharacterized protein C14orf119",
  "gene_symbol": "C14orf119",
  "gene": "UniProtKB:Q9NWQ9",
  "term_label": "Unknown cellular component"
}